{
  "gene": "UniProtKB:Q9UNH5",
  "gene_symbol": "CDC14A",
  "term_id": "GO:0060271",
  "gene_name": "Dual specificity protein phosphatase CDC14A",
  "term_label": "cilium assembly"
}